{
  "term_id": "GO:0003735",
  "gene": "UniProtKB:P82675",
  "gene_name": "Small ribosomal subunit protein uS5m",
  "gene_symbol": "MRPS5",
  "term_label": "structural constituent of ribosome"
}